aluminum ion transmembrane transport [GO:1902602] (biological process) Definition: The directed movement of aluminium ions across a membrane. Relationships: is a type of transmembrane transport [GO:0055085] Also known as: aluminium transmembrane transport, aluminum transmembrane transport, aluminium ion transmembrane transport Sources: GOC:TermGenie, GOC:pr, GO_REF:0000069